{
  "gene_symbol": "AOX1",
  "term_id": "UNKNOWN:0002",
  "gene_name": "Aldehyde oxidase",
  "gene": "UniProtKB:Q06278",
  "term_label": "Unknown biological process"
}